phenylpropanoid metabolic process [GO:0009698] (biological process) Definition: The chemical reactions and pathways involving aromatic derivatives of trans-cinnamic acid. Regulation: RO_0002211 by regulation of phenylpropanoid metabolic process [GO:2000762] Also known as: phenylpropanoid metabolism Subtypes: GO:0009699, cinnamic acid ester metabolic process [GO:0009801], cinnamic acid metabolic process [GO:0009803], GO:0009804, lignan metabolic process [GO:0009806], lignin metabolic process [GO:0009808], GO:0042854, phenylpropanoid catabolic process [GO:0046271], isoflavonoid metabolic process [GO:0046287] Sources: GOC:jl Relationships: is a type of secondary metabolic process [GO:0019748]